very-long-chain (3R)-3-hydroxyacyl-CoA dehydratase activity [GO:0102158] (molecular function) References: PMID:16564093, PMID:19763486 Sources: RHEA:45812 Also known as: very-long-chain 3-hydroxyacyl-CoA dehydratase activity Relationships: is a type of (2E)-enoyl-CoA hydratase activity [GO:0080023] Definition: Catalysis of the reaction: a very-long-chain (3R)-3-hydroxyacyl-CoA = H2O + a very-long-chain (2E)-enoyl-CoA. This reaction is the third (dehydration) step of the four-step fatty acid elongation cycle in the endoplasmic reticulum that extends fatty acids of C-16 or longer with an additional 2-C unit.